{
  "gene": "UniProtKB:Q9UP79",
  "gene_symbol": "ADAMTS8",
  "term_label": "extracellular matrix organization",
  "gene_name": "A disintegrin and metalloproteinase with thrombospondin motifs 8",
  "term_id": "GO:0030198"
}